{
  "gene": "UniProtKB:Q9UH77",
  "term_label": "monoatomic ion homeostasis",
  "gene_symbol": "KLHL3",
  "term_id": "GO:0050801",
  "gene_name": "Kelch-like protein 3"
}